{
  "term_label": "Unknown molecular function",
  "term_id": "UNKNOWN:0001",
  "gene_symbol": "PRR23D1",
  "gene": "UniProtKB:E9PI22",
  "gene_name": "Proline-rich protein 23D1"
}